{
  "term_label": "Unknown cellular component",
  "gene_name": "cGMP-specific 3',5'-cyclic phosphodiesterase",
  "gene_symbol": "PDE5A",
  "term_id": "UNKNOWN:0003",
  "gene": "UniProtKB:O76074"
}